{
  "gene_symbol": "ZC4H2",
  "term_label": "nucleus",
  "gene": "UniProtKB:Q9NQZ6",
  "gene_name": "Zinc finger C4H2 domain-containing protein",
  "term_id": "GO:0005634"
}